{
  "gene_name": "Spindle assembly abnormal protein 6 homolog",
  "term_id": "GO:0007283",
  "gene_symbol": "SASS6",
  "gene": "UniProtKB:Q6UVJ0",
  "term_label": "spermatogenesis"
}